{
  "term_label": "external side of plasma membrane",
  "gene": "UniProtKB:Q7KYR7",
  "term_id": "GO:0009897",
  "gene_symbol": "BTN2A1",
  "gene_name": "Butyrophilin subfamily 2 member A1"
}